neuron differentiation [GO:0030182] (biological process) Sources: GOC:mah Relationships: is a type of cell differentiation [GO:0030154]; is part of GO:0048699 Definition: The process in which a relatively unspecialized cell acquires specialized features of a neuron. Subtypes: noradrenergic neuron differentiation [GO:0003357], GO:0003387, GO:0021526, GO:0021953, GO:0035315, GO:0042490, GO:0046530, peripheral nervous system neuron differentiation [GO:0048934], neuron differentiation involved in salivary gland development [GO:0060705], neuroendocrine cell differentiation [GO:0061101], dopaminergic neuron differentiation [GO:0071542], GABAergic neuron differentiation [GO:0097154], glutamatergic neuron differentiation [GO:1905962] Regulation: regulated by GO:0045664; negatively regulated by negative regulation of neuron differentiation [GO:0045665]; positively regulated by GO:0045666